positive regulation of leucophore differentiation [GO:0048777] (biological process) Definition: Any process that activates or increases the frequency, rate or extent of leucophore differentiation. Also known as: up regulation of leucophore differentiation, up-regulation of leucophore differentiation, upregulation of leucophore differentiation, activation of leucophore differentiation, stimulation of leucophore differentiation Sources: GOC:mh Relationships: is a type of regulation of leucophore differentiation [GO:0048775]; is a type of positive regulation of pigment cell differentiation [GO:0050942]; positively regulates leucophore differentiation [GO:0048772]